{
  "term_label": "U7 snRNP",
  "gene": "UniProtKB:P83369",
  "gene_name": "U7 snRNA-associated Sm-like protein LSm11",
  "term_id": "GO:0005683",
  "gene_symbol": "LSM11"
}